{
  "gene": "UniProtKB:P00995",
  "gene_name": "Serine protease inhibitor Kazal-type 1",
  "term_id": "UNKNOWN:0002",
  "term_label": "Unknown biological process",
  "gene_symbol": "SPINK1"
}